{
  "gene_name": "rRNA methyltransferase 3, mitochondrial",
  "term_id": "UNKNOWN:0001",
  "gene": "UniProtKB:Q9HC36",
  "gene_symbol": "MRM3",
  "term_label": "Unknown molecular function"
}